{
  "term_label": "midbody",
  "term_id": "GO:0030496",
  "gene_symbol": "CEP126",
  "gene": "UniProtKB:Q9P2H0",
  "gene_name": "Centrosomal protein of 126 kDa"
}